{
  "term_id": "GO:0050877",
  "gene": "UniProtKB:Q9UHB7",
  "term_label": "nervous system process",
  "gene_name": "AF4_FMR2 family member 4",
  "gene_symbol": "AFF4"
}